RNA methylation [GO:0001510] (biological process) Definition: Posttranscriptional addition of a methyl group to either a nucleotide or 2'-O ribose in a polyribonucleotide. Usually uses S-adenosylmethionine as a cofactor. References: PMID:21823225 Sources: GOC:hjd Subtypes: tRNA methylation [GO:0030488], rRNA methylation [GO:0031167], 7-methylguanosine cap hypermethylation [GO:0036261], RNA (guanine-N7)-methylation [GO:0036265], snRNA methylation [GO:0106349] Relationships: is a type of GO:0009451; is a type of macromolecule methylation [GO:0043414]